cellular response to laminar fluid shear stress [GO:0071499] (biological process) Sources: GOC:mah Definition: Any process that results in a change in state or activity of a cell (in terms of movement, secretion, enzyme production, gene expression, etc.) as a result of a laminar fluid shear stress stimulus. Laminar fluid flow is the force acting on an object in a system where the fluid is moving across a solid surface in parallel layers. Subtypes: vascular endothelial cell response to laminar fluid shear stress [GO:0097700] Relationships: is a type of response to laminar fluid shear stress [GO:0034616]; is a type of cellular response to fluid shear stress [GO:0071498]